{
  "gene_name": "Sodium leak channel NALCN",
  "term_label": "positive regulation of synaptic transmission, GABAergic",
  "gene": "UniProtKB:Q8IZF0",
  "term_id": "GO:0032230",
  "gene_symbol": "NALCN"
}